O-acyltransferase activity [GO:0008374] (molecular function) Subtypes: ecdysone O-acyltransferase activity [GO:0004173], GO:0004366, phosphatidylcholine-sterol O-acyltransferase activity [GO:0004607], sterol O-acyltransferase activity [GO:0004772], GO:0008779, acyl-[acyl-carrier-protein]-UDP-N-acetylglucosamine O-acyltransferase activity [GO:0008780], carnitine O-acyltransferase activity [GO:0016406], acylglycerol O-acyltransferase activity [GO:0016411], serine O-acyltransferase activity [GO:0016412], O-acetyltransferase activity [GO:0016413], diglucosylglycerate octanoyltransferase activity [GO:0016414], O-palmitoyltransferase activity [GO:0016416], O-succinyltransferase activity [GO:0016750], GO:0016753, GO:0032216, O-linoleoyltransferase activity [GO:0032576], alcohol O-acyltransferase activity [GO:0034318], 2-acylglycerol-3-phosphate O-acyltransferase activity [GO:0047144], plasmalogen synthase activity [GO:0047159], 1-alkenylglycerophosphoethanolamine O-acyltransferase activity [GO:0047166], 1-alkyl-2-acetylglycerol O-acyltransferase activity [GO:0047167], phosphatidylcholine-retinol O-acyltransferase activity [GO:0047173], galactosylacylglycerol O-acyltransferase activity [GO:0047175], 1-acylglycerophosphocholine O-acyltransferase activity [GO:0047184], 2-acylglycerophosphocholine O-acyltransferase activity [GO:0047190], 1-alkylglycerophosphocholine O-acyltransferase activity [GO:0047191], indoleacetylglucose-inositol O-acyltransferase activity [GO:0047194], diacylglycerol-sterol O-acyltransferase activity [GO:0047195], long-chain-alcohol O-fatty-acyltransferase activity [GO:0047196], triglyceride-sterol O-acyltransferase activity [GO:0047197], phosphatidylcholine-dolichol O-acyltransferase activity [GO:0047199], dolichol O-acyltransferase activity [GO:0047872], GO:0047909, GO:0050252, O-malonyltransferase activity [GO:0050736], O-hydroxycinnamoyltransferase activity [GO:0050737], GO:0080095, phosphatidate-sterol O-acyltransferase activity [GO:0080096], glycerol-3-phosphate 2-O-acyltransferase activity [GO:0090447], 1-acylglycerophosphoethanolamine O-acyltransferase activity [GO:0106262], 1-acylglycerophosphoserine O-acyltransferase activity [GO:0106263] Relationships: is a type of GO:0016747 Definition: Catalysis of the transfer of an acyl group to an oxygen atom on the acceptor molecule. Sources: GOC:ai